{
  "term_label": "serine-type endopeptidase inhibitor activity",
  "gene_symbol": "SERPINB9",
  "gene": "UniProtKB:P50453",
  "term_id": "GO:0004867",
  "gene_name": "Serpin B9"
}